{
  "term_id": "GO:0061511",
  "gene": "UniProtKB:Q9HC77",
  "term_label": "centriole elongation",
  "gene_name": "Centromere protein J",
  "gene_symbol": "CENPJ"
}